regulation of locomotion [GO:0040012] (biological process) Sources: GOC:ems Subtypes: negative regulation of locomotion [GO:0040013], positive regulation of locomotion [GO:0040017], regulation of backward locomotion [GO:0043058], GO:0043059, regulation of chemotaxis [GO:0050920], regulation of locomotion involved in locomotory behavior [GO:0090325], regulation of cell motility [GO:2000145] Definition: Any process that modulates the frequency, rate or extent of locomotion of a cell or organism. Relationships: is a type of regulation of biological process [GO:0050789]; regulates locomotion [GO:0040011]